{
  "gene_name": "Receptor tyrosine-protein kinase erbB-4",
  "gene": "UniProtKB:Q15303",
  "term_label": "epidermal growth factor receptor binding",
  "term_id": "GO:0005154",
  "gene_symbol": "ERBB4"
}